{
  "gene_name": "IGF-like family receptor 1",
  "term_label": "Unknown molecular function",
  "gene": "UniProtKB:Q9H665",
  "term_id": "UNKNOWN:0001",
  "gene_symbol": "IGFLR1"
}